{
  "gene": "UniProtKB:P07225",
  "gene_name": "Vitamin K-dependent protein S",
  "term_label": "negative regulation of coagulation",
  "term_id": "GO:0050819",
  "gene_symbol": "PROS1"
}